{
  "term_id": "GO:0015629",
  "gene_name": "Calponin-3",
  "gene": "UniProtKB:Q15417",
  "gene_symbol": "CNN3",
  "term_label": "actin cytoskeleton"
}